{
  "gene": "UniProtKB:Q8TF61",
  "gene_symbol": "FBXO41",
  "term_id": "UNKNOWN:0001",
  "term_label": "Unknown molecular function",
  "gene_name": "F-box only protein 41"
}